regulation of acetylcholine biosynthetic process [GO:1905921] (biological process) Relationships: is_a GO:0009889; is a type of GO:0060408; regulates GO:0008292 Definition: Any process that modulates the frequency, rate or extent of acetylcholine biosynthetic process. Also known as: regulation of acetylcholine anabolism, regulation of acetylcholine biosynthesis, regulation of acetylcholine formation, regulation of acetylcholine synthesis References: PMID:20164328 Sources: GOC:TermGenie, GOC:aruk, GOC:bc, GO_REF:0000058 Subtypes: negative regulation of acetylcholine biosynthetic process [GO:1905922], GO:1905923